{
  "gene": "UniProtKB:Q7Z3Z0",
  "gene_symbol": "KRT25",
  "term_id": "GO:0005856",
  "term_label": "cytoskeleton",
  "gene_name": "Keratin, type I cytoskeletal 25"
}